negative regulation of myeloid dendritic cell cytokine production [GO:0002734] (biological process) Relationships: is a type of GO:0002731; is a type of regulation of myeloid dendritic cell cytokine production [GO:0002733]; is a type of negative regulation of myeloid leukocyte mediated immunity [GO:0002887]; negatively regulates myeloid dendritic cell cytokine production [GO:0002372] Sources: GOC:add Definition: Any process that stops, prevents, or reduces the frequency, rate, or extent of myeloid dendritic cell cytokine production. Also known as: down regulation of myeloid dendritic cell cytokine production, down-regulation of myeloid dendritic cell cytokine production, downregulation of myeloid dendritic cell cytokine production, inhibition of myeloid dendritic cell cytokine production